{
  "term_id": "GO:0004725",
  "gene_name": "Receptor-type tyrosine-protein phosphatase F",
  "gene_symbol": "PTPRF",
  "gene": "UniProtKB:P10586",
  "term_label": "protein tyrosine phosphatase activity"
}